{
  "gene_name": "Tetratricopeptide repeat protein 14",
  "gene_symbol": "TTC14",
  "term_label": "Unknown molecular function",
  "gene": "UniProtKB:Q96N46",
  "term_id": "UNKNOWN:0001"
}